{
  "gene_symbol": "DMBX1",
  "gene_name": "Diencephalon_mesencephalon homeobox protein 1",
  "gene": "UniProtKB:Q8NFW5",
  "term_id": "GO:0000981",
  "term_label": "DNA-binding transcription factor activity, RNA polymerase II-specific"
}